{
  "gene_symbol": "PRDM7",
  "term_id": "UNKNOWN:0001",
  "gene_name": "Histone-lysine N-methyltransferase PRDM7",
  "term_label": "Unknown molecular function",
  "gene": "UniProtKB:Q9NQW5"
}